fatty acid derivative metabolic process [GO:1901568] (biological process) Also known as: fatty acid derivative metabolism Sources: GOC:TermGenie, GOC:pr Definition: The chemical reactions and pathways involving fatty acid derivative. Relationships: is a type of lipid metabolic process [GO:0006629] Subtypes: wax metabolic process [GO:0010166], protocatechuate catabolic process, ortho-cleavage [GO:0019618], fatty-acyl-CoA metabolic process [GO:0035337], leukotriene B4 metabolic process [GO:0036102], GO:0062126, fatty acid derivative catabolic process [GO:1901569], fatty acid derivative biosynthetic process [GO:1901570], leukotriene A4 metabolic process [GO:1901751], ketone body metabolic process [GO:1902224], fatty acid methyl ester metabolic process [GO:1902898], fatty alcohol metabolic process [GO:1903173], lipoxin A4 metabolic process [GO:2001302], lipoxin B4 metabolic process [GO:2001304]